{
  "term_label": "cytosol",
  "term_id": "GO:0005829",
  "gene_symbol": "SPRY1",
  "gene": "UniProtKB:O43609",
  "gene_name": "Protein sprouty homolog 1"
}